{
  "gene_name": "B-cell lymphoma_leukemia 11B",
  "gene": "UniProtKB:Q9C0K0",
  "term_id": "GO:0045944",
  "term_label": "positive regulation of transcription by RNA polymerase II",
  "gene_symbol": "BCL11B"
}